{
  "term_label": "signaling receptor complex adaptor activity",
  "gene_symbol": "SPAG9",
  "gene": "UniProtKB:O60271",
  "term_id": "GO:0030159",
  "gene_name": "C-Jun-amino-terminal kinase-interacting protein 4"
}